{
  "term_id": "GO:0046935",
  "term_label": "1-phosphatidylinositol-3-kinase regulator activity",
  "gene": "UniProtKB:O00459",
  "gene_name": "Phosphatidylinositol 3-kinase regulatory subunit beta",
  "gene_symbol": "PIK3R2"
}